{
  "gene": "UniProtKB:Q92750",
  "gene_name": "Transcription initiation factor TFIID subunit 4B",
  "term_label": "DNA binding",
  "term_id": "GO:0003677",
  "gene_symbol": "TAF4B"
}